{
  "gene_name": "Selenoprotein M",
  "term_label": "Unknown biological process",
  "gene_symbol": "SELENOM",
  "term_id": "UNKNOWN:0002",
  "gene": "UniProtKB:Q8WWX9"
}